cross-receptor inhibition within G protein-coupled receptor heterodimer [GO:0038041] (biological process) References: PMID:15979374 Sources: GOC:al, GOC:bf Definition: Inhibition of one protomer of a G protein-coupled receptor (GPCR) heterodimer by the associated subunit. For example, agonist activation of one cytokine receptor can prevent activation of its associated cytokine receptor subunit. Relationships: is a type of regulation of G protein-coupled receptor signaling pathway [GO:0008277]; is a type of negative regulation of signaling receptor activity [GO:2000272] Also known as: cross-receptor inhibition within G-protein coupled receptor heterodimer